smooth muscle tissue development [GO:0048745] (biological process) Sources: GOC:dph, GOC:jid, GOC:lm Relationships: is a type of muscle tissue development [GO:0060537] Definition: The process whose specific outcome is the progression of smooth muscle over time, from its formation to the mature structure. Regulation: regulated by regulation of smooth muscle tissue development [GO:1905899]; negatively regulated by negative regulation of smooth muscle tissue development [GO:1905900]; positively regulated by GO:1905901 Subtypes: GO:0061145, GO:0072191, GO:0072194